{
  "gene": "UniProtKB:Q6ZN66",
  "term_label": "GTPase activity",
  "gene_symbol": "GBP6",
  "term_id": "GO:0003924",
  "gene_name": "Guanylate-binding protein 6"
}